{
  "gene_symbol": "CORT",
  "term_label": "extracellular space",
  "term_id": "GO:0005615",
  "gene": "UniProtKB:O00230",
  "gene_name": "Cortistatin"
}